{
  "term_label": "Unknown biological process",
  "gene_symbol": "LY6G5B",
  "gene": "UniProtKB:Q8NDX9",
  "gene_name": "Lymphocyte antigen 6 complex locus protein G5b",
  "term_id": "UNKNOWN:0002"
}